{
  "term_label": "cell fate commitment",
  "gene_symbol": "GATA2",
  "gene_name": "Endothelial transcription factor GATA-2",
  "term_id": "GO:0045165",
  "gene": "UniProtKB:P23769"
}